{
  "gene_symbol": "NKD1",
  "gene_name": "Protein naked cuticle homolog 1",
  "gene": "UniProtKB:Q969G9",
  "term_id": "GO:0005737",
  "term_label": "cytoplasm"
}